{
  "term_id": "GO:0015842",
  "gene_name": "Chromaffin granule amine transporter",
  "term_label": "aminergic neurotransmitter loading into synaptic vesicle",
  "gene": "UniProtKB:P54219",
  "gene_symbol": "SLC18A1"
}